regulation of intracellular signal transduction [GO:1902531] (biological process) Sources: GOC:TermGenie, GOC:dph, GOC:signaling, GOC:tb Relationships: is a type of GO:0009966; regulates intracellular signal transduction [GO:0035556] Definition: Any process that modulates the frequency, rate or extent of intracellular signal transduction. Also known as: regulation of intracellular signaling cascade, regulation of intracellular signaling chain, regulation of intracellular protein kinase cascade, regulation of intracellular signal transduction pathway, regulation of signal transmission via intracellular cascade, regulation of intracellular signaling pathway, regulation of signal transduction via intracellular signaling cascade Subtypes: GO:0002155, regulation of nitric oxide mediated signal transduction [GO:0010749], GO:0032006, regulation of intracellular steroid hormone receptor signaling pathway [GO:0033143], regulation of hippo signaling [GO:0035330], regulation of peroxisome proliferator activated receptor signaling pathway [GO:0035358], regulation of cytoplasmic pattern recognition receptor signaling pathway [GO:0039531], regulation of canonical NF-kappaB signal transduction [GO:0043122], GO:0043408, GO:0048385, GO:0050848, regulation of small GTPase mediated signal transduction [GO:0051056], regulation of phosphatidylinositol 3-kinase/protein kinase B signal transduction [GO:0051896], regulation of SMAD protein signal transduction [GO:0060390], regulation of phosphorelay signal transduction system [GO:0070297], GO:0070302, regulation of vitamin D receptor signaling pathway [GO:0070562], regulation of protein kinase C signaling [GO:0090036], regulation of cAMP/PKA signal transduction [GO:0141161], GO:1900101, regulation of non-canonical NF-kappaB signal transduction [GO:1901222], regulation of signal transduction by p53 class mediator [GO:1901796], regulation of cell cycle checkpoint [GO:1901976], regulation of hypoxia-inducible factor-1alpha signaling pathway [GO:1902071], GO:1902532, positive regulation of intracellular signal transduction [GO:1902533], GO:2000638, regulation of intrinsic apoptotic signaling pathway [GO:2001242]